{
  "gene_symbol": "NCOA1",
  "gene_name": "Nuclear receptor coactivator 1",
  "term_id": "GO:0005634",
  "term_label": "nucleus",
  "gene": "UniProtKB:Q15788"
}